establishment of natural killer cell polarity [GO:0001770] (biological process) References: PMID:12615886, PMID:9759849 Sources: GOC:mgi_curators Also known as: NK cell polarization, establishment of NK cell polarity, natural killer cell polarization Relationships: is a type of establishment of lymphocyte polarity [GO:0001767]; is part of natural killer cell activation [GO:0030101] Definition: The directed orientation of natural killer cell signaling molecules and associated membrane rafts towards a chemokine gradient or a contact point with a cell displaying natural killer cell activating ligands.